{
  "gene_symbol": "LINC00482",
  "gene_name": "Putative uncharacterized protein encoded by LINC00482",
  "gene": "UniProtKB:Q8N8I6",
  "term_label": "Unknown molecular function",
  "term_id": "UNKNOWN:0001"
}